{
  "gene_name": "Cadherin-13",
  "term_id": "GO:0000902",
  "gene_symbol": "CDH13",
  "term_label": "cell morphogenesis",
  "gene": "UniProtKB:P55290"
}